{
  "term_id": "GO:0005634",
  "gene_symbol": "APOBEC2",
  "gene": "UniProtKB:Q9Y235",
  "term_label": "nucleus",
  "gene_name": "C-U-editing enzyme APOBEC-2"
}